{
  "gene_symbol": "EHHADH",
  "gene_name": "Peroxisomal bifunctional enzyme",
  "gene": "UniProtKB:Q08426",
  "term_id": "GO:0005777",
  "term_label": "peroxisome"
}